ent-sandaracopimaradiene synthase activity [GO:0034280] (molecular function) Sources: RHEA:25536 Definition: Catalysis of the reaction: ent-copalyl diphosphate = ent-sandaracopimara-8(14),15-diene + diphosphate. Relationships: is a type of GO:0016838 Also known as: ent-pimaradiene synthase activity, ent-copalyl-diphosphate diphosphate-lyase [ent-sandaracopimara-8(14),15-diene-forming] activity